{
  "term_id": "GO:0005834",
  "gene": "UniProtKB:O60262",
  "term_label": "heterotrimeric G-protein complex",
  "gene_name": "Guanine nucleotide-binding protein G(I)_G(S)_G(O) subunit gamma-7",
  "gene_symbol": "GNG7"
}